positive regulation of response to cytokine stimulus [GO:0060760] (biological process) Definition: Any process that increases the rate, frequency, or extent of a response to cytokine stimulus. Relationships: is a type of positive regulation of response to stimulus [GO:0048584]; is a type of regulation of response to cytokine stimulus [GO:0060759]; RO_0002213 response to cytokine [GO:0034097] Sources: GOC:BHF, GOC:dph, GOC:tb Subtypes: positive regulation of cytokine-mediated signaling pathway [GO:0001961], positive regulation of response to type II interferon [GO:0060332], positive regulation of response to macrophage colony-stimulating factor [GO:1903971]